{
  "gene": "UniProtKB:P23246",
  "gene_name": "Splicing factor, proline- and glutamine-rich",
  "term_label": "alternative mRNA splicing, via spliceosome",
  "gene_symbol": "SFPQ",
  "term_id": "GO:0000380"
}